{
  "term_id": "GO:0005789",
  "gene_name": "Translocating chain-associated membrane protein 2",
  "gene": "UniProtKB:Q15035",
  "term_label": "endoplasmic reticulum membrane",
  "gene_symbol": "TRAM2"
}